positive regulation of octopamine signaling pathway [GO:2000130] (biological process) Sources: GOC:mah Also known as: positive regulation of octopamine signalling pathway Definition: Any process that activates or increases the frequency, rate or extent of octopamine signaling pathway. Relationships: is a type of positive regulation of octopamine or tyramine signaling pathway [GO:2000127]; is_a regulation of octopamine signaling pathway [GO:2000128]; positively regulates octopamine signaling pathway [GO:0071927] Subtypes: positive regulation of octopamine signaling pathway involved in response to food [GO:2000141]